phagolysosome membrane [GO:0061474] (cellular component) References: PMID:22073313 Sources: GOC:dph Definition: The lipid bilayer surrounding a phagolysosome. Relationships: is a type of lysosomal membrane [GO:0005765]; is a type of phagocytic vesicle membrane [GO:0030670]; is part of phagolysosome [GO:0032010]